negative regulation of amyloid precursor protein biosynthetic process [GO:0042985] (biological process) Definition: Any process that stops, prevents, or reduces the frequency, rate or extent of the chemical reactions and pathways resulting in the formation of amyloid precursor protein (APP), the precursor of amyloid-beta. Sources: GOC:go_curators Also known as: down regulation of amyloid precursor protein biosynthetic process, down-regulation of amyloid precursor protein biosynthetic process, downregulation of amyloid precursor protein biosynthetic process, negative regulation of APP biosynthesis, negative regulation of APP biosynthetic process, negative regulation of amyloid precursor protein anabolism, negative regulation of amyloid precursor protein biosynthesis, negative regulation of amyloid precursor protein formation, negative regulation of amyloid precursor protein synthesis, inhibition of amyloid precursor protein biosynthetic process Relationships: is a type of GO:0010561; is a type of regulation of amyloid precursor protein biosynthetic process [GO:0042984]; negatively regulates amyloid precursor protein biosynthetic process [GO:0042983]